nicotinamide-nucleotide amidase activity [GO:0019159] (molecular function) Definition: Catalysis of the reaction: beta-nicotinamide D-ribonucleotide + H2O = beta-nicotinate D-ribonucleotide + NH3. Also known as: NMN amidohydrolase, NMN deamidase activity, nicotinamide mononucleotide amidohydrolase activity, nicotinamide mononucleotide deamidase activity, nicotinamide-D-ribonucleotide amidohydrolase activity Sources: EC:3.5.1.42 Relationships: is a type of hydrolase activity, acting on carbon-nitrogen (but not peptide) bonds, in linear amides [GO:0016811]